{
  "term_id": "GO:0005886",
  "term_label": "plasma membrane",
  "gene_symbol": "OR2T4",
  "gene_name": "Olfactory receptor 2T4",
  "gene": "UniProtKB:Q8NH00"
}